{
  "gene_symbol": "SOX4",
  "gene": "UniProtKB:Q06945",
  "gene_name": "Transcription factor SOX-4",
  "term_id": "GO:0030182",
  "term_label": "neuron differentiation"
}